chlorate transmembrane transporter activity [GO:0015107] (molecular function) Definition: Enables the transfer of chlorate, ClO3-, from one side of a membrane to the other. Relationships: is a type of GO:0022857; is part of chlorate transport [GO:0015702] Sources: GOC:curators